{
  "gene_symbol": "RAP1GAP2",
  "term_id": "GO:0030424",
  "gene_name": "Rap1 GTPase-activating protein 2",
  "term_label": "axon",
  "gene": "UniProtKB:Q684P5"
}